mediator complex binding [GO:0036033] (molecular function) Relationships: is a type of protein-containing complex binding [GO:0044877] Definition: Binding to a mediator complex. The mediator complex is a protein complex that interacts with the carboxy-terminal domain of the largest subunit of RNA polymerase II and plays an active role in transducing the signal from a transcription factor to the transcriptional machinery. The Saccharomyces complex contains several identifiable subcomplexes: a head domain comprising Srb2, -4, and -5, Med6, -8, and -11, and Rox3 proteins; a middle domain comprising Med1, -4, and -7, Nut1 and -2, Cse2, Rgr1, Soh1, and Srb7 proteins; a tail consisting of Gal11p, Med2p, Pgd1p, and Sin4p; and a regulatory subcomplex comprising Ssn2, -3, and -8, and Srb8 proteins. Metazoan mediator complexes have similar modular structures and include homologs of yeast Srb and Med proteins. References: PMID:18391015 Sources: GOC:yaf